sarcosine oxidase complex [GO:0032921] (cellular component) Definition: A complex consisting of 4 protein subunits as a heterotetramer, that possesses sarcosine oxidase activity. Relationships: is a type of oxidoreductase complex [GO:1990204]; is part of cytoplasm [GO:0005737] Sources: GOC:mah, GOC:mlg